hydrolase activity, acting on ether bonds [GO:0016801] (molecular function) Sources: GOC:ai, GOC:jl Subtypes: GO:0016802, ether hydrolase activity [GO:0016803] Definition: Catalysis of the hydrolysis of any ether or thioether bond, -O- or -S- respectively. Relationships: is a type of GO:0016787